{
  "gene_symbol": "CTLA4",
  "gene": "UniProtKB:P16410",
  "gene_name": "Cytotoxic T-lymphocyte protein 4",
  "term_label": "T cell receptor signaling pathway",
  "term_id": "GO:0050852"
}